andrastin A biosynthetic process [GO:0140876] (biological process) Also known as: andrastin A anabolism, andrastin A biosynthesis, andrastin A formation, andrastin A synthesis Sources: DOI:10.1016/j.tet.2013.07.029 Relationships: is a type of steroid biosynthetic process [GO:0006694]; is a type of ketone biosynthetic process [GO:0042181]; is a type of mycotoxin biosynthetic process [GO:0043386]; is a type of aldehyde biosynthetic process [GO:0046184]; is a type of GO:0120255 Definition: The chemical reactions and pathways resulting in the formation of andrastin A, a meroterpenoid that exhibits inhibitory activity against ras farnesyltransferase, suggesting that it could have promising antitumor activity.